{
  "term_label": "respiratory chain complex IV",
  "term_id": "GO:0045277",
  "gene_symbol": "NDUFA4L2",
  "gene": "UniProtKB:Q9NRX3",
  "gene_name": "NADH dehydrogenase [ubiquinone] 1 alpha subcomplex subunit 4-like 2"
}